{
  "term_id": "GO:0008119",
  "gene": "UniProtKB:P51580",
  "gene_name": "Thiopurine S-methyltransferase",
  "term_label": "thiopurine S-methyltransferase activity",
  "gene_symbol": "TPMT"
}